lysophospholipid translocation [GO:0140329] (biological process) References: PMID:15661733 Definition: The movement of a lysophospholipid molecule from one leaflet of a membrane bilayer to the opposite leaflet. Relationships: is a type of GO:0045332; is a type of lysophospholipid transport [GO:0051977]